{
  "gene_symbol": "ACOXL",
  "gene_name": "Acyl-coenzyme A oxidase-like protein",
  "term_label": "fatty acid binding",
  "gene": "UniProtKB:Q9NUZ1",
  "term_id": "GO:0005504"
}